{
  "term_id": "GO:0007018",
  "term_label": "microtubule-based movement",
  "gene_symbol": "KIF19",
  "gene_name": "Kinesin-like protein KIF19",
  "gene": "UniProtKB:Q2TAC6"
}